{
  "gene_name": "Apolipoprotein C-I",
  "term_id": "GO:0032375",
  "gene_symbol": "APOC1",
  "gene": "UniProtKB:P02654",
  "term_label": "negative regulation of cholesterol transport"
}